{
  "gene": "UniProtKB:Q8NCQ7",
  "term_label": "Unknown cellular component",
  "gene_symbol": "PROCA1",
  "term_id": "UNKNOWN:0003",
  "gene_name": "Protein PROCA1"
}